DNA damage tolerance [GO:0006301] (biological process) Relationships: is a type of DNA metabolic process [GO:0006259]; is a type of GO:0006974; is part of DNA replication [GO:0006260] Also known as: postreplication DNA repair, postreplication repair References: PMID:18157158, PMID:26322163, PMID:31251805 Definition: A process that promotes the bypass of single-stranded DNA lesions encountered by DNA polymerases during DNA replication, thereby preventing replication fork stalling and allowing completion of DNA replication without removing the damage. Subtypes: translesion synthesis [GO:0019985], error-free postreplication DNA repair [GO:0042275]